{
  "gene_symbol": "PURB",
  "gene": "UniProtKB:Q96QR8",
  "term_id": "GO:0005634",
  "term_label": "nucleus",
  "gene_name": "Transcriptional activator protein Pur-beta"
}